{
  "gene": "UniProtKB:O15481",
  "term_id": "GO:0000122",
  "gene_symbol": "MAGEB4",
  "gene_name": "Melanoma-associated antigen B4",
  "term_label": "negative regulation of transcription by RNA polymerase II"
}